{
  "gene": "UniProtKB:P62070",
  "gene_symbol": "RRAS2",
  "gene_name": "Ras-related protein R-Ras2",
  "term_label": "Ras protein signal transduction",
  "term_id": "GO:0007265"
}